{
  "term_id": "UNKNOWN:0002",
  "gene": "UniProtKB:A0A024RCN7",
  "term_label": "Unknown biological process",
  "gene_name": "Chromosome 6 open reading frame 48, isoform CRA_a",
  "gene_symbol": "SNHG32"
}